positive regulation of blood coagulation, common pathway [GO:2000262] (biological process) Relationships: is a type of positive regulation of blood coagulation [GO:0030194]; is_a positive regulation of protein activation cascade [GO:2000259]; is a type of regulation of blood coagulation, common pathway [GO:2000260]; positively regulates blood coagulation, common pathway [GO:0072377] Definition: Any process that activates or increases the frequency, rate or extent of blood coagulation, common pathway. Sources: GOC:mah